regulation of long-term synaptic depression [GO:1900452] (biological process) Definition: Any process that modulates the frequency, rate or extent of long term synaptic depression. Sources: GOC:BHF, GOC:TermGenie Subtypes: negative regulation of long-term synaptic depression [GO:1900453], positive regulation of long-term synaptic depression [GO:1900454] Also known as: regulation of long term depression, regulation of long term synaptic depression, regulation of LTD Relationships: is a type of regulation of synaptic plasticity [GO:0048167]; regulates GO:0060292